negative regulation of biosynthetic process of antibacterial peptides active against Gram-negative bacteria [GO:0002814] (biological process) Definition: Any process that stops, prevents, or reduces the frequency, rate, or extent of biosynthesis of antibacterial peptides active against Gram-negative bacteria. Also known as: down regulation of biosynthetic process of antibacterial peptides active against Gram-negative bacteria, down-regulation of biosynthetic process of antibacterial peptides active against Gram-negative bacteria, downregulation of biosynthetic process of antibacterial peptides active against Gram-negative bacteria, inhibition of biosynthetic process of antibacterial peptides active against Gram-negative bacteria Relationships: is a type of negative regulation of antibacterial peptide biosynthetic process [GO:0002809]; is a type of regulation of biosynthetic process of antibacterial peptides active against Gram-negative bacteria [GO:0002813]; negatively regulates biosynthetic process of antibacterial peptides active against Gram-negative bacteria [GO:0002812] Sources: GOC:add